{
  "gene_symbol": "UBE2F",
  "gene": "UniProtKB:Q969M7",
  "term_label": "protein neddylation",
  "gene_name": "NEDD8-conjugating enzyme UBE2F",
  "term_id": "GO:0045116"
}